{
  "term_id": "GO:0050728",
  "term_label": "negative regulation of inflammatory response",
  "gene_name": "Nuclear receptor ROR-alpha",
  "gene_symbol": "RORA",
  "gene": "UniProtKB:P35398"
}